{
  "gene_symbol": "OR9G1",
  "term_label": "Unknown biological process",
  "term_id": "UNKNOWN:0002",
  "gene_name": "Olfactory receptor 9G1",
  "gene": "UniProtKB:Q8NH87"
}